D-glutamyltransferase activity [GO:0047823] (molecular function) Also known as: D-gamma-glutamyl transpeptidase activity, D-glutamyl transpeptidase activity, glutamine:D-glutamyl-peptide 5-glutamyltransferase activity Definition: Catalysis of the reaction: D-glutamate + D-glutamine = gamma-D-glutamyl-D-glutamate + NH4+. Can also transfer additional glutamyl residues to a peptide, extending the polypeptide chain. Sources: EC:2.3.2.1 Relationships: is a type of GO:0016755